positive regulation of prostaglandin secretion involved in immune response [GO:0061078] (BP) Definition: Any process that activates or increases the frequency, rate or extent of the regulated release of a prostaglandin from a cell and contributes to the immune response. Sources: GOC:BHF, GOC:dph Relationships: is a type of positive regulation of prostaglandin secretion [GO:0032308]; positively regulates GO:0090323 Also known as: positive regulation of prostaglandin secretion during immune response